{
  "term_id": "GO:0001228",
  "gene_name": "Transcription factor SOX-12",
  "gene": "UniProtKB:O15370",
  "term_label": "DNA-binding transcription activator activity, RNA polymerase II-specific",
  "gene_symbol": "SOX12"
}